{
  "gene_symbol": "DCST1",
  "gene_name": "E3 ubiquitin-protein ligase DCST1",
  "gene": "UniProtKB:Q5T197",
  "term_label": "Unknown biological process",
  "term_id": "UNKNOWN:0002"
}